{
  "gene_name": "Brother of CDO",
  "gene_symbol": "BOC",
  "term_label": "axon",
  "term_id": "GO:0030424",
  "gene": "UniProtKB:Q9BWV1"
}